{
  "gene": "UniProtKB:Q05952",
  "term_label": "acrosome reaction",
  "term_id": "GO:0007340",
  "gene_name": "Nuclear transition protein 2",
  "gene_symbol": "TNP2"
}